{
  "gene": "UniProtKB:O14786",
  "term_id": "GO:0048010",
  "gene_symbol": "NRP1",
  "term_label": "vascular endothelial growth factor receptor signaling pathway",
  "gene_name": "Neuropilin-1"
}